{
  "gene_symbol": "UNC50",
  "term_label": "Unknown molecular function",
  "gene": "UniProtKB:Q53HI1",
  "gene_name": "Protein unc-50 homolog",
  "term_id": "UNKNOWN:0001"
}